{
  "gene": "UniProtKB:P26717",
  "term_label": "positive regulation of natural killer cell mediated cytotoxicity",
  "gene_symbol": "KLRC2",
  "term_id": "GO:0045954",
  "gene_name": "NKG2-C type II integral membrane protein"
}